{
  "gene": "UniProtKB:Q9NQT8",
  "gene_name": "Kinesin-like protein KIF13B",
  "gene_symbol": "KIF13B",
  "term_id": "GO:0005874",
  "term_label": "microtubule"
}